{
  "gene": "UniProtKB:Q16656",
  "term_id": "GO:0005634",
  "gene_symbol": "NRF1",
  "term_label": "nucleus",
  "gene_name": "Nuclear respiratory factor 1"
}